{
  "gene": "UniProtKB:P27658",
  "gene_name": "Collagen alpha-1(VIII) chain",
  "term_label": "extracellular matrix organization",
  "gene_symbol": "COL8A1",
  "term_id": "GO:0030198"
}